{
  "gene": "UniProtKB:Q5TA89",
  "gene_name": "Transcription factor HES-5",
  "term_id": "GO:0050767",
  "term_label": "regulation of neurogenesis",
  "gene_symbol": "HES5"
}